positive regulation of G0 to G1 transition [GO:0070318] (biological process) Relationships: is a type of regulation of G0 to G1 transition [GO:0070316]; is a type of positive regulation of cell cycle process [GO:0090068]; RO_0002213 GO:0045023 Definition: A cell cycle process that activates or increases the rate or extent of the transition from the G0 quiescent state to the G1 phase. Sources: GOC:mah